{
  "term_label": "Unknown molecular function",
  "gene": "UniProtKB:Q96M89",
  "gene_symbol": "CCDC138",
  "gene_name": "Coiled-coil domain-containing protein 138",
  "term_id": "UNKNOWN:0001"
}